lithium ion transport [GO:0010351] (BP) Subtypes: GO:0090452 References: PMID:17270011 Relationships: is a type of metal ion transport [GO:0030001] Also known as: lithium transport Definition: The directed movement of lithium ion into, out of or within a cell, or between cells, by means of some agent such as a transporter or pore.